{
  "gene_symbol": "SMO",
  "term_id": "GO:0005886",
  "gene": "UniProtKB:Q99835",
  "gene_name": "Protein smoothened",
  "term_label": "plasma membrane"
}